{
  "term_id": "GO:0007274",
  "gene_symbol": "CHRNB3",
  "gene": "UniProtKB:Q05901",
  "term_label": "neuromuscular synaptic transmission",
  "gene_name": "Neuronal acetylcholine receptor subunit beta-3"
}